{
  "gene": "UniProtKB:Q9Y2I7",
  "gene_name": "1-phosphatidylinositol 3-phosphate 5-kinase",
  "gene_symbol": "PIKFYVE",
  "term_label": "cytoplasmic vesicle",
  "term_id": "GO:0031410"
}